{
  "gene_symbol": "ADSL",
  "term_label": "N6-(1,2-dicarboxyethyl)AMP AMP-lyase (fumarate-forming) activity",
  "term_id": "GO:0004018",
  "gene": "UniProtKB:P30566",
  "gene_name": "Adenylosuccinate lyase"
}